{
  "term_id": "UNKNOWN:0003",
  "term_label": "Unknown cellular component",
  "gene_name": "Diphthine--ammonia ligase",
  "gene": "UniProtKB:Q7L8W6",
  "gene_symbol": "DPH6"
}